{
  "gene_name": "Zinc finger C2HC domain-containing protein 1C",
  "term_label": "Unknown biological process",
  "term_id": "UNKNOWN:0002",
  "gene_symbol": "ZC2HC1C",
  "gene": "UniProtKB:Q53FD0"
}